{
  "gene_name": "Protein phosphatase 1 regulatory subunit 1B",
  "term_id": "GO:0035556",
  "term_label": "intracellular signal transduction",
  "gene_symbol": "PPP1R1B",
  "gene": "UniProtKB:Q9UD71"
}